{
  "term_label": "Unknown biological process",
  "gene_symbol": "LUM",
  "gene_name": "Lumican",
  "term_id": "UNKNOWN:0002",
  "gene": "UniProtKB:P51884"
}